{
  "term_id": "UNKNOWN:0001",
  "term_label": "Unknown molecular function",
  "gene_symbol": "GAREM2",
  "gene_name": "GRB2-associated and regulator of MAPK protein 2",
  "gene": "UniProtKB:Q75VX8"
}